{
  "gene": "UniProtKB:Q15428",
  "gene_symbol": "SF3A2",
  "term_label": "spliceosomal complex assembly",
  "gene_name": "Splicing factor 3A subunit 2",
  "term_id": "GO:0000245"
}